phragmoplast [GO:0009524] (cellular component) References: PMID:28943203 Relationships: is a type of cellular anatomical structure [GO:0110165]; is part of cytoplasm [GO:0005737] Definition: The phragmoplast is a plant cell specific cytoplasmic structure composed of cytoskeletal polymers, membranes, and associated cytosolic proteins that functions as the focused secretory module for assembling the cell plate.